{
  "gene_symbol": "AQP7",
  "term_id": "GO:0015254",
  "gene_name": "Aquaporin-7",
  "term_label": "glycerol channel activity",
  "gene": "UniProtKB:O14520"
}